negative regulation of long-term synaptic potentiation [GO:1900272] (biological process) Relationships: is_a negative regulation of biological process [GO:0048519]; is a type of regulation of long-term synaptic potentiation [GO:1900271]; negatively regulates long-term synaptic potentiation [GO:0060291] Sources: GOC:BHF, GOC:TermGenie Definition: Any process that stops, prevents or reduces the frequency, rate or extent of long-term synaptic potentiation. Also known as: down regulation of long-term potentiation, down-regulation of long-term potentiation, downregulation of long-term potentiation, inhibition of long-term potentiation, negative regulation of long-term potentiation, down regulation of long-term synaptic potentiation, down-regulation of long-term synaptic potentiation, downregulation of long-term synaptic potentiation, inhibition of long-term synaptic potentiation, down regulation of LTP, down-regulation of LTP, downregulation of LTP, inhibition of LTP, negative regulation of LTP